oculomotor nerve development [GO:0021557] (BP) Sources: GOC:cls, GOC:dgh, GOC:dph, GOC:jid, GO_REF:0000021 Definition: The process whose specific outcome is the progression of the oculomotor nerve over time, from its formation to the mature structure. This motor nerve innervates all extraocular muscles except the superior oblique and the lateral rectus muscles. The superior division supplies the levator palpebrae superioris and superior rectus muscles. The inferior division supplies the medial rectus, inferior rectus and inferior oblique muscles. This nerve also innervates the striated muscles of the eyelid. Pupillary constriction and lens movement are mediated by this nerve for near vision. In the orbit the inferior division sends branches that enter the ciliary ganglion where they form functional contacts (synapses) with the ganglion cells. The ganglion cells send nerve fibers into the back of the eye where they travel to ultimately innervate the ciliary muscle and the constrictor pupillae muscle. Also known as: cranial nerve 3 development, cranial nerve III development, CN III development Relationships: is a type of cranial nerve development [GO:0021545]; is part of preganglionic parasympathetic fiber development [GO:0021783]